caveola bulb [GO:0099401] (cellular component) Relationships: is a type of membrane microdomain [GO:0098857] References: PMID:17227843 Sources: GOC:PARL, GOC:POD Also known as: caveola crater Definition: The region of a caveola that extends into the cytoplasm, excluding the neck (rim). This region is associated with intracellular caveola proteins.